{
  "gene_symbol": "SLC25A45",
  "term_label": "Unknown biological process",
  "term_id": "UNKNOWN:0002",
  "gene": "UniProtKB:Q8N413",
  "gene_name": "Solute carrier family 25 member 45"
}